{
  "gene": "UniProtKB:Q9Y277",
  "gene_symbol": "VDAC3",
  "gene_name": "Voltage-dependent anion-selective channel protein 3",
  "term_label": "mitochondrial outer membrane",
  "term_id": "GO:0005741"
}